{
  "term_id": "UNKNOWN:0003",
  "gene": "UniProtKB:Q96F10",
  "gene_name": "Thialysine N-epsilon-acetyltransferase",
  "gene_symbol": "SAT2",
  "term_label": "Unknown cellular component"
}